{
  "gene_name": "Synaptojanin-1",
  "gene": "UniProtKB:O43426",
  "term_id": "GO:0048488",
  "gene_symbol": "SYNJ1",
  "term_label": "synaptic vesicle endocytosis"
}